{
  "gene_symbol": "BBOF1",
  "term_id": "UNKNOWN:0002",
  "gene": "UniProtKB:Q8ND07",
  "gene_name": "Basal body-orientation factor 1",
  "term_label": "Unknown biological process"
}